vesicle cytoskeletal trafficking [GO:0099518] (BP) Relationships: is a type of cytoskeleton-dependent intracellular transport [GO:0030705]; is a type of establishment of vesicle localization [GO:0051650] Definition: The directed movement of a vesicle along a cytoskeletal fiber such as a microtubule or and actin filament, mediated by motor proteins. Subtypes: GO:0030050, vesicle transport along microtubule [GO:0047496], synaptic vesicle cytoskeletal transport [GO:0099514], dense core granule cytoskeletal transport [GO:0099519] Also known as: cytoskeletal fiber-based vesicle localization, vesicle cytoskeletal transport Sources: GOC:ecd, GOC:rl